{
  "term_id": "GO:0005634",
  "gene": "UniProtKB:O77932",
  "gene_name": "Decapping and exoribonuclease protein",
  "gene_symbol": "DXO",
  "term_label": "nucleus"
}